hypotonic response [GO:0006971] (BP) Relationships: is a type of response to osmotic stress [GO:0006970] References: PMID:12598593 Sources: GOC:jl Subtypes: GO:0042539, cellular hypotonic response [GO:0071476] Definition: Any process that results in a change in state or activity of a cell or an organism (in terms of movement, secretion, enzyme production, gene expression, etc.) as a result of detection of, or exposure to, a hypotonic environment, i.e. an environment with a lower concentration of solutes than the organism or cell. Also known as: hypo-osmotic response